{
  "term_id": "GO:0050839",
  "gene": "UniProtKB:O60500",
  "gene_symbol": "NPHS1",
  "term_label": "cell adhesion molecule binding",
  "gene_name": "Nephrin"
}